{
  "gene_symbol": "IER5",
  "term_label": "Unknown molecular function",
  "gene_name": "Immediate early response gene 5 protein",
  "gene": "UniProtKB:Q5VY09",
  "term_id": "UNKNOWN:0001"
}